{
  "term_label": "Unknown molecular function",
  "gene_symbol": "TMEM108",
  "gene_name": "Transmembrane protein 108",
  "term_id": "UNKNOWN:0001",
  "gene": "UniProtKB:Q6UXF1"
}